{
  "term_id": "GO:0043303",
  "gene": "UniProtKB:Q7Z7G1",
  "gene_name": "Cytokine-dependent hematopoietic cell linker",
  "gene_symbol": "CLNK",
  "term_label": "mast cell degranulation"
}